{
  "term_label": "response to insulin",
  "gene_name": "Ketohexokinase",
  "gene": "UniProtKB:P50053",
  "term_id": "GO:0032868",
  "gene_symbol": "KHK"
}